TAP2 binding [GO:0046979] (molecular function) Relationships: is a type of GO:0046977 Definition: Binding to the TAP2 subunit of TAP (transporter associated with antigen processing) protein. References: PMID:11133832